{
  "gene_symbol": "YIPF4",
  "gene": "UniProtKB:Q9BSR8",
  "gene_name": "Protein YIPF4",
  "term_label": "vesicle fusion with Golgi apparatus",
  "term_id": "GO:0048280"
}